{
  "term_id": "UNKNOWN:0001",
  "term_label": "Unknown molecular function",
  "gene": "UniProtKB:Q9Y4F9",
  "gene_symbol": "RIPOR2",
  "gene_name": "Rho family-interacting cell polarization regulator 2"
}